{
  "term_label": "endoplasmic reticulum exit site",
  "gene": "UniProtKB:O95487",
  "term_id": "GO:0070971",
  "gene_name": "Protein transport protein Sec24B",
  "gene_symbol": "SEC24B"
}